{
  "gene_symbol": "HP1BP3",
  "term_label": "nucleus",
  "gene": "UniProtKB:Q5SSJ5",
  "term_id": "GO:0005634",
  "gene_name": "Heterochromatin protein 1-binding protein 3"
}